{
  "gene_symbol": "KIR2DL5B",
  "gene": "UniProtKB:Q8NHK3",
  "term_id": "GO:0005886",
  "gene_name": "Killer cell immunoglobulin-like receptor 2DL5B",
  "term_label": "plasma membrane"
}